{
  "term_id": "GO:0031588",
  "gene": "UniProtKB:P54646",
  "gene_symbol": "PRKAA2",
  "term_label": "nucleotide-activated protein kinase complex",
  "gene_name": "5'-AMP-activated protein kinase catalytic subunit alpha-2"
}